{
  "term_label": "intracellular protein transport",
  "term_id": "GO:0006886",
  "gene_symbol": "TMED9",
  "gene": "UniProtKB:Q9BVK6",
  "gene_name": "Transmembrane emp24 domain-containing protein 9"
}